{
  "gene": "UniProtKB:Q6PKG0",
  "term_label": "cytosol",
  "term_id": "GO:0005829",
  "gene_symbol": "LARP1",
  "gene_name": "La-related protein 1"
}